{
  "term_id": "GO:0048812",
  "gene_name": "Unconventional myosin-XVI",
  "gene": "UniProtKB:Q9Y6X6",
  "term_label": "neuron projection morphogenesis",
  "gene_symbol": "MYO16"
}